{
  "gene_name": "Interleukin-1 receptor-associated kinase-like 2",
  "gene_symbol": "IRAK2",
  "term_id": "GO:0008063",
  "term_label": "Toll signaling pathway",
  "gene": "UniProtKB:O43187"
}